{
  "term_id": "GO:0000981",
  "gene": "UniProtKB:Q969W8",
  "term_label": "DNA-binding transcription factor activity, RNA polymerase II-specific",
  "gene_name": "Zinc finger protein 566",
  "gene_symbol": "ZNF566"
}